hair follicle placode formation [GO:0060789] (biological process) Definition: The developmental process in which a hair placode forms. An hair follicle placode is a thickening of the ectoderm that will give rise to the hair follicle bud. Sources: GOC:dph, GOC:sdb_2009, GOC:tb Relationships: is a type of ectodermal placode formation [GO:0060788]; is part of hair follicle development [GO:0001942] Regulation: regulated by regulation of hair follicle placode formation [GO:0061168]; positively regulated by positive regulation of hair placode formation [GO:0061169]; negatively regulated by negative regulation of hair follicle placode formation [GO:0061170]